{
  "term_id": "GO:0045717",
  "gene": "UniProtKB:Q8N5D0",
  "term_label": "negative regulation of fatty acid biosynthetic process",
  "gene_name": "WD and tetratricopeptide repeats protein 1",
  "gene_symbol": "WDTC1"
}